{
  "term_label": "calcium ion binding",
  "term_id": "GO:0005509",
  "gene_symbol": "EFHD1",
  "gene": "UniProtKB:Q9BUP0",
  "gene_name": "EF-hand domain-containing protein D1"
}